{
  "gene": "UniProtKB:Q9C0D7",
  "gene_name": "Probable ribonuclease ZC3H12C",
  "term_label": "mRNA binding",
  "term_id": "GO:0003729",
  "gene_symbol": "ZC3H12C"
}